{
  "gene_name": "Inositol-trisphosphate 3-kinase A",
  "gene": "UniProtKB:P23677",
  "term_label": "nucleus",
  "term_id": "GO:0005634",
  "gene_symbol": "ITPKA"
}